{
  "term_label": "Unknown biological process",
  "gene_symbol": "APOL2",
  "gene": "UniProtKB:Q9BQE5",
  "gene_name": "Apolipoprotein L2",
  "term_id": "UNKNOWN:0002"
}